{
  "gene_name": "Zinc finger protein 3 homolog",
  "gene_symbol": "ZFP3",
  "gene": "UniProtKB:Q96NJ6",
  "term_label": "DNA-binding transcription factor activity, RNA polymerase II-specific",
  "term_id": "GO:0000981"
}